negative regulation of monodictyphenone biosynthetic process [GO:1900844] (biological process) Relationships: is_a negative regulation of small molecule metabolic process [GO:0062014]; is a type of negative regulation of secondary metabolite biosynthetic process [GO:1900377]; is a type of regulation of monodictyphenone biosynthetic process [GO:1900843]; RO_0002212 GO:1900815 Also known as: down regulation of monodictyphenone biosynthetic process, down-regulation of monodictyphenone biosynthetic process, downregulation of monodictyphenone biosynthetic process Sources: GOC:TermGenie, GOC:di Definition: Any process that stops, prevents or reduces the frequency, rate or extent of monodictyphenone biosynthetic process.